{
  "gene_name": "Ras-related protein Rab-7a",
  "term_id": "UNKNOWN:0001",
  "term_label": "Unknown molecular function",
  "gene_symbol": "RAB7A",
  "gene": "UniProtKB:P51149"
}